semaphorin receptor activity [GO:0017154] (molecular function) References: PMID:15239958 Sources: GOC:mah, GOC:signaling Definition: Combining with a semaphorin, and transmitting the signal from one side of the membrane to the other to initiate a change in cell activity. Relationships: is a type of transmembrane signaling receptor activity [GO:0004888]; is part of semaphorin-plexin signaling pathway [GO:0071526]